renal system pattern specification [GO:0072048] (biological process) Relationships: is a type of pattern specification process [GO:0007389]; is part of renal system development [GO:0072001] Subtypes: renal system segmentation [GO:0061150], metanephric cap specification [GO:0072188] Definition: Any developmental process that results in the creation of defined areas or spaces within an organism to which cells respond and eventually are instructed to differentiate into the anatomical structures of the renal system. Sources: GOC:mtg_kidney_jan10 Also known as: renal system pattern formation